miRNA catabolic process [GO:0010587] (biological process) References: PMID:17993620 Relationships: is a type of RNA catabolic process [GO:0006401]; is a type of miRNA metabolic process [GO:0010586] Definition: The chemical reactions and pathways resulting in the breakdown of miRNA, microRNA, a class of single-stranded RNA molecules of about 21-23 nucleotides in length, which regulates gene expression. Regulation: regulated by regulation of miRNA catabolic process [GO:2000625]; negatively regulated by negative regulation of miRNA catabolic process [GO:2000626]; positively regulated by GO:2000627 Subtypes: target-directed miRNA degradation [GO:0140958] Also known as: microRNA catabolic process